posterior midgut development [GO:0007497] (biological process) Sources: GOC:go_curators Relationships: is a type of GO:0048856; is part of midgut development [GO:0007494] Definition: The process whose specific outcome is the progression of the posterior midgut over time, from its formation to the mature structure.